heart rudiment development [GO:0003313] (biological process) Definition: The progression of the heart rudiment over time, from its initial formation to the mature structure. The heart rudiment is a cone-like structure that is formed when myocardial progenitor cells of the heart field fuse at the midline. The heart rudiment is the first structure of the heart tube. Sources: GOC:mtg_heart Relationships: is a type of epithelium development [GO:0060429]; is part of embryonic heart tube development [GO:0035050] Also known as: heart cone development